aliphatic desulfoglucosinolate sulfotransferase activity [GO:0120527] (molecular function) Relationships: is a type of sulfotransferase activity [GO:0008146] Definition: Catalysis of the reaction: 3'-phosphoadenylyl sulfate + an aliphatic (Z)-desulfo-glucosinolate = a (Z)-omega-(methylsulfanyl)-N-sulfo-alkylhydroximate S-glucoside + adenosine 3',5'-bisphosphate + H+. Sources: RHEA:52724